cellular response to abiotic stimulus [GO:0071214] (biological process) Definition: Any process that results in a change in state or activity of a cell (in terms of movement, secretion, enzyme production, gene expression, etc.) as a result of an abiotic (non-living) stimulus. Sources: GOC:mah Also known as: cellular response to abiotic stress Note: Note that this term is in the subset of terms that should not be used for direct gene product annotation. Instead, select a child term or, if no appropriate child term exists, please request a new term. Direct annotations to this term may be amended during annotation QC. Relationships: is a type of GO:0009628; is a type of cellular response to environmental stimulus [GO:0104004] Subtypes: GO:0071257, cellular response to gravity [GO:0071258], cellular response to magnetism [GO:0071259], GO:0071260, cellular response to water stimulus [GO:0071462], cellular response to pH [GO:0071467], cellular response to osmotic stress [GO:0071470], GO:0071478, cellular response to viscosity [GO:0097715]